{
  "gene_symbol": "PRPF3",
  "term_id": "UNKNOWN:0001",
  "term_label": "Unknown molecular function",
  "gene_name": "U4_U6 small nuclear ribonucleoprotein Prp3",
  "gene": "UniProtKB:O43395"
}